free ubiquitin chain depolymerization [GO:0010995] (biological process) Definition: The process in which free ubiquitin chains, compounds composed of a large number of ubiquitin monomers, are broken down. Sources: GOC:BHF, GOC:dph, GOC:tb Relationships: is a type of protein depolymerization [GO:0051261]; is part of ubiquitin recycling [GO:0010992]